{
  "term_label": "positive regulation of B cell differentiation",
  "gene": "UniProtKB:Q92835",
  "gene_symbol": "INPP5D",
  "gene_name": "Phosphatidylinositol 3,4,5-trisphosphate 5-phosphatase 1",
  "term_id": "GO:0045579"
}